{
  "term_label": "RNA polymerase II cis-regulatory region sequence-specific DNA binding",
  "gene_name": "Pituitary-specific positive transcription factor 1",
  "term_id": "GO:0000978",
  "gene_symbol": "POU1F1",
  "gene": "UniProtKB:P28069"
}